polytene chromosome interband [GO:0005705] (cellular component) References: PMID:11361342 Sources: GOC:bf Definition: A stretch of less tightly packed chromatin along the polytene chromosome, found between bands. Relationships: is a type of GO:0098687; is part of polytene chromosome [GO:0005700]